{
  "term_id": "UNKNOWN:0001",
  "gene_name": "Formin-binding protein 4",
  "gene_symbol": "FNBP4",
  "term_label": "Unknown molecular function",
  "gene": "UniProtKB:Q8N3X1"
}